{
  "gene": "UniProtKB:Q9Y2U5",
  "gene_symbol": "MAP3K2",
  "term_id": "GO:0000165",
  "gene_name": "Mitogen-activated protein kinase kinase kinase 2",
  "term_label": "MAPK cascade"
}